negative regulation of vasoconstriction [GO:0045906] (biological process) Sources: GOC:go_curators Definition: Any process that stops, prevents, or reduces the frequency, rate or extent of vasoconstriction. Relationships: is a type of regulation of vasoconstriction [GO:0019229]; is a type of negative regulation of multicellular organismal process [GO:0051241]; RO_0002212 vasoconstriction [GO:0042310] Also known as: down regulation of vasoconstriction, down-regulation of vasoconstriction, downregulation of vasoconstriction, inhibition of vasoconstriction Subtypes: negative regulation of vascular associated smooth muscle contraction [GO:1904694]